{
  "gene_name": "Mitochondrial import receptor subunit TOM20 homolog",
  "term_id": "GO:0030150",
  "term_label": "protein import into mitochondrial matrix",
  "gene": "UniProtKB:Q15388",
  "gene_symbol": "TOMM20"
}